{
  "gene_symbol": "CACNA2D2",
  "term_label": "voltage-gated calcium channel activity",
  "gene": "UniProtKB:Q9NY47",
  "term_id": "GO:0005245",
  "gene_name": "Voltage-dependent calcium channel subunit alpha-2_delta-2"
}